nervous system process [GO:0050877] (biological process) Regulation: regulated by regulation of nervous system process [GO:0031644]; negatively regulated by GO:0031645; RO_0002213 by positive regulation of nervous system process [GO:0031646] Subtypes: nervous system process involved in regulation of systemic arterial blood pressure [GO:0001976], detection of dietary excess [GO:0002022], regulation of respiratory gaseous exchange by nervous system process [GO:0002087], sensory perception [GO:0007600], transmission of nerve impulse [GO:0019226], GO:0019227, cognition [GO:0050890], neuromuscular process [GO:0050905], detection of mechanical stimulus involved in sensory perception of sound [GO:0050910], echolocation [GO:0050959], GO:0071066, cerebrospinal fluid circulation [GO:0090660], GO:0099531, GO:0099565 Also known as: neurological system process, neurophysiological process, pan-neural process Definition: An organ system process carried out by any of the organs or tissues of the neurological system. Relationships: is a type of system process [GO:0003008] Sources: GOC:ai, GOC:mtg_cardio